{
  "gene_name": "NF-kappa-B inhibitor-like protein 1",
  "term_id": "UNKNOWN:0001",
  "term_label": "Unknown molecular function",
  "gene_symbol": "NFKBIL1",
  "gene": "UniProtKB:Q9UBC1"
}